{
  "term_label": "mRNA splicing, via spliceosome",
  "gene": "UniProtKB:Q9Y333",
  "term_id": "GO:0000398",
  "gene_name": "U6 snRNA-associated Sm-like protein LSm2",
  "gene_symbol": "LSM2"
}